tergite morphogenesis [GO:0007490] (biological process) References: PMID:16451739 Sources: GOC:jid Relationships: is_a post-embryonic animal morphogenesis [GO:0009886]; is part of histoblast morphogenesis [GO:0007488] Definition: The process in which the anatomical structures of the tergite are generated and organized. The tergite is the primary plate or sclerite forming the dorsal surface of any insect body segment.